{
  "gene_name": "Proline-rich protein 11",
  "term_label": "Unknown biological process",
  "gene": "UniProtKB:Q96HE9",
  "gene_symbol": "PRR11",
  "term_id": "UNKNOWN:0002"
}